{
  "gene_symbol": "MYH13",
  "term_id": "GO:0051015",
  "gene_name": "Myosin-13",
  "gene": "UniProtKB:Q9UKX3",
  "term_label": "actin filament binding"
}